{
  "term_label": "frizzled binding",
  "gene_name": "Protein Wnt-5b",
  "gene": "UniProtKB:Q9H1J7",
  "gene_symbol": "WNT5B",
  "term_id": "GO:0005109"
}